{
  "gene_name": "Sodium_glucose cotransporter 2",
  "gene": "UniProtKB:P31639",
  "term_id": "GO:0098708",
  "gene_symbol": "SLC5A2",
  "term_label": "D-glucose import across plasma membrane"
}